negative regulation of mesenchymal to epithelial transition involved in mesonephros morphogenesis [GO:2000085] (biological process) Relationships: is a type of GO:2000084; is_a negative regulation of epithelial cell differentiation involved in kidney development [GO:2000697]; negatively regulates GO:0061261 Sources: GOC:mtg_kidney_jan10 Definition: Any process that stops, prevents, or reduces the frequency, rate or extent of mesenchymal to epithelial transition involved in mesonephros morphogenesis. Also known as: negative regulation of mesonephric mesenchyme to epithelial transition